valine metabolic process [GO:0006573] (biological process) Subtypes: GO:0006574, L-valine biosynthetic process [GO:0009099], D-valine metabolic process [GO:1902114] Relationships: is a type of branched-chain amino acid metabolic process [GO:0009081]; is a type of alpha-amino acid metabolic process [GO:1901605] Definition: The chemical reactions and pathways involving valine, 2-amino-3-methylbutanoic acid. Sources: GOC:ai Also known as: valine metabolism